7,8-didemethyl-8-hydroxy-5-deazariboflavin synthase complex [GO:0044673] (cellular component) Definition: A heterodimer which catalyses the reaction of 5-amino-6-(D-ribitylamino)uracil and 4-hydroxyphenylpyruvate to form 7,8-didemethyl-8-hydroxy-5-deazariboflavin (FO), an intermediate of coenzyme F420. References: PMID:14593448 Sources: GOC:mengo_curators Also known as: FO-synthase complex Relationships: is_a catalytic complex [GO:1902494]